{
  "term_id": "GO:0005793",
  "gene_name": "Nucleobindin-1",
  "gene_symbol": "NUCB1",
  "term_label": "endoplasmic reticulum-Golgi intermediate compartment",
  "gene": "UniProtKB:Q02818"
}